tetrahydrocolumbamine 2-O-methyltransferase activity [GO:0030762] (molecular function) Sources: EC:2.1.1.89, RHEA:22536 Definition: Catalysis of the reaction: (S)-tetrahydrocolumbamine + S-adenosyl-L-methionine(1+) = S-adenosyl-L-homocysteine + H+ + tetrahydropalmatine. Also known as: S-adenosyl-L-methionine:5,8,13,13a-tetrahydrocolumbamine 2-O-methyltransferase activity, tetrahydrocolumbamine methyltransferase activity Relationships: is a type of GO:0008757